{
  "gene_symbol": "TINF2",
  "term_label": "regulation of telomere maintenance via telomere lengthening",
  "gene_name": "TERF1-interacting nuclear factor 2",
  "gene": "UniProtKB:Q9BSI4",
  "term_id": "GO:1904356"
}